protein-lipid complex remodeling [GO:0034368] (biological process) Subtypes: GO:0034369 Relationships: is a type of protein-containing complex remodeling [GO:0034367]; is a type of protein-lipid complex organization [GO:0071825] Definition: The acquisition, loss or modification of a protein or lipid within a protein-lipid complex. Sources: GOC:BHF, GOC:mah, GOC:rl Also known as: protein-lipid complex remodelling